virion maturation [GO:0098677] (biological process) Sources: ISBN:0781718325, VZ:1946 Also known as: viral particle maturation, virus particle maturation Relationships: is a type of GO:0016032; is part of virus maturation [GO:0019075] Definition: Maturation of a virion after separation from the host cell. Not all viruses mature after separation. In those that do, maturation typically involves rearangement and/or cleavage of viral proteins, resulting in the virion becoming competent for reinfection.